{
  "gene_symbol": "TMOD3",
  "gene_name": "Tropomodulin-3",
  "term_label": "myofibril assembly",
  "gene": "UniProtKB:Q9NYL9",
  "term_id": "GO:0030239"
}